{
  "term_id": "GO:0031883",
  "gene_symbol": "REEP2",
  "gene_name": "Receptor expression-enhancing protein 2",
  "gene": "UniProtKB:Q9BRK0",
  "term_label": "taste receptor binding"
}